{
  "gene": "UniProtKB:Q9BXS6",
  "term_id": "GO:0008017",
  "gene_symbol": "NUSAP1",
  "gene_name": "Nucleolar and spindle-associated protein 1",
  "term_label": "microtubule binding"
}